{
  "term_id": "GO:0005096",
  "term_label": "GTPase activator activity",
  "gene_symbol": "ARHGAP11A",
  "gene": "UniProtKB:Q6P4F7",
  "gene_name": "Rho GTPase-activating protein 11A"
}